egg chorion assembly [GO:0007306] (biological process) Definition: Construction of the chorion portion of the egg, which is a protective, noncellular membrane that surrounds the eggs of various animals including insects and fish. References: PMID:24804966 Sources: GOC:dph, GOC:mtg_sensu, GOC:tb, ISBN:0879694238 Also known as: eggshell chorion formation, insect chorion formation Relationships: is a type of developmental process involved in reproduction [GO:0003006]; is a type of cellular component assembly involved in morphogenesis [GO:0010927]; is a type of cellular process involved in reproduction in multicellular organism [GO:0022412]; is a type of external encapsulating structure organization [GO:0045229]